{
  "term_id": "GO:0051056",
  "gene_name": "Rho GTPase-activating protein 18",
  "term_label": "regulation of small GTPase mediated signal transduction",
  "gene_symbol": "ARHGAP18",
  "gene": "UniProtKB:Q8N392"
}